{
  "term_label": "Unknown biological process",
  "gene_name": "Coiled-coil domain-containing protein 43",
  "gene_symbol": "CCDC43",
  "gene": "UniProtKB:Q96MW1",
  "term_id": "UNKNOWN:0002"
}